{
  "term_id": "GO:0005682",
  "gene": "UniProtKB:P62318",
  "gene_name": "Small nuclear ribonucleoprotein Sm D3",
  "gene_symbol": "SNRPD3",
  "term_label": "U5 snRNP"
}